regulation of smooth muscle cell migration [GO:0014910] (biological process) Relationships: is a type of regulation of cell migration [GO:0030334]; regulates GO:0014909 Sources: CL:0000192, GOC:mtg_muscle Subtypes: positive regulation of smooth muscle cell migration [GO:0014911], GO:0014912, regulation of smooth muscle cell chemotaxis [GO:0071671], regulation of vascular associated smooth muscle cell migration [GO:1904752] Definition: Any process that modulates the frequency, rate or extent of smooth muscle cell migration.